{
  "gene_name": "Equilibrative nucleobase transporter 1",
  "gene": "UniProtKB:Q8NBI5",
  "gene_symbol": "SLC43A3",
  "term_label": "Unknown cellular component",
  "term_id": "UNKNOWN:0003"
}